{
  "gene_symbol": "ICE1",
  "term_label": "snRNA transcription by RNA polymerase II",
  "gene": "UniProtKB:Q9Y2F5",
  "term_id": "GO:0042795",
  "gene_name": "Little elongation complex subunit 1"
}